asynchronous neurotransmitter secretion [GO:0071912] (biological process) Definition: Release of neurotransmitter at the synapse that persists for tens to hundreds of milliseconds after action potential invasion. References: PMID:19477156, PMID:20643933 Sources: GOC:dsf Relationships: is a type of GO:0007269